{
  "gene": "UniProtKB:A8K855",
  "term_id": "GO:0060170",
  "gene_name": "EF-hand calcium-binding domain-containing protein 7",
  "term_label": "ciliary membrane",
  "gene_symbol": "EFCAB7"
}